T cell differentiation in thymus [GO:0033077] (BP) Note: Note that immunologists typically use the word 'development' to refer to cells of B or T cell lineages undergoing the process that GO describes as 'cell differentiation'. Regulation: regulated by regulation of T cell differentiation in thymus [GO:0033081]; negatively regulated by negative regulation of T cell differentiation in thymus [GO:0033085]; positively regulated by GO:0033089 Relationships: is a type of GO:0030217 Definition: The process in which a precursor cell type acquires the specialized features of a T cell via a differentiation pathway dependent upon transit through the thymus. Also known as: thymic T cell differentiation, thymocyte cell differentiation, thymocyte differentiation, T cell development in thymus Subtypes: DN2 thymocyte differentiation [GO:1904155], GO:1904156, DN4 thymocyte differentiation [GO:1904157] Sources: GOC:add, ISBN:0781735149